{
  "gene": "UniProtKB:Q14566",
  "gene_symbol": "MCM6",
  "term_id": "GO:0005634",
  "gene_name": "DNA replication licensing factor MCM6",
  "term_label": "nucleus"
}